{
  "term_id": "UNKNOWN:0002",
  "gene_name": "Cilia- and flagella-associated protein 77",
  "term_label": "Unknown biological process",
  "gene": "UniProtKB:Q6ZQR2",
  "gene_symbol": "CFAP77"
}